{
  "term_label": "activin receptor activity, type I",
  "gene_name": "Activin receptor type-1B",
  "gene": "UniProtKB:P36896",
  "term_id": "GO:0016361",
  "gene_symbol": "ACVR1B"
}